{
  "gene_symbol": "HSD17B6",
  "term_label": "Unknown cellular component",
  "gene_name": "17-beta-hydroxysteroid dehydrogenase type 6",
  "term_id": "UNKNOWN:0003",
  "gene": "UniProtKB:O14756"
}